{
  "term_id": "UNKNOWN:0001",
  "term_label": "Unknown molecular function",
  "gene_name": "Putative tetratricopeptide repeat protein 41",
  "gene_symbol": "TTC41P",
  "gene": "UniProtKB:Q6P2S7"
}